{
  "gene": "UniProtKB:Q5VTT5",
  "gene_symbol": "MYOM3",
  "term_label": "structural constituent of muscle",
  "term_id": "GO:0008307",
  "gene_name": "Myomesin-3"
}